{
  "gene": "UniProtKB:Q92828",
  "gene_symbol": "CORO2A",
  "term_id": "GO:0051015",
  "term_label": "actin filament binding",
  "gene_name": "Coronin-2A"
}